{
  "gene_name": "Metallothionein-3",
  "term_label": "cellular response to cadmium ion",
  "term_id": "GO:0071276",
  "gene_symbol": "MT3",
  "gene": "UniProtKB:P25713"
}